{
  "term_id": "GO:0000981",
  "gene_symbol": "CASZ1",
  "gene": "UniProtKB:Q86V15",
  "gene_name": "Zinc finger protein castor homolog 1",
  "term_label": "DNA-binding transcription factor activity, RNA polymerase II-specific"
}